{
  "term_id": "UNKNOWN:0001",
  "gene_symbol": "POLR3GL",
  "gene": "UniProtKB:Q9BT43",
  "gene_name": "DNA-directed RNA polymerase III subunit RPC7-like",
  "term_label": "Unknown molecular function"
}